{
  "gene_symbol": "OR4M2B",
  "gene_name": "Olfactory receptor 4M2",
  "gene": "UniProtKB:A0A0X1KG70",
  "term_id": "GO:0005886",
  "term_label": "plasma membrane"
}